{
  "gene": "UniProtKB:P10075",
  "gene_name": "Zinc finger protein GLI4",
  "term_label": "RNA polymerase II cis-regulatory region sequence-specific DNA binding",
  "term_id": "GO:0000978",
  "gene_symbol": "GLI4"
}